{
  "gene_name": "Oligodendrocyte-myelin glycoprotein",
  "gene_symbol": "OMG",
  "term_id": "UNKNOWN:0003",
  "gene": "UniProtKB:P23515",
  "term_label": "Unknown cellular component"
}